{
  "term_id": "GO:0009617",
  "gene_symbol": "TRAV39",
  "term_label": "response to bacterium",
  "gene_name": "T cell receptor alpha variable 39",
  "gene": "UniProtKB:A0A0B4J263"
}